{
  "term_id": "GO:0000978",
  "gene": "UniProtKB:O95475",
  "gene_name": "Homeobox protein SIX6",
  "term_label": "RNA polymerase II cis-regulatory region sequence-specific DNA binding",
  "gene_symbol": "SIX6"
}